{
  "gene_symbol": "SPRY1",
  "gene": "UniProtKB:O43609",
  "term_id": "GO:0046580",
  "gene_name": "Protein sprouty homolog 1",
  "term_label": "negative regulation of Ras protein signal transduction"
}